ascending aorta morphogenesis [GO:0035910] (biological process) Sources: GOC:bf, GOC:dgh, MA:0002570, UBERON:0001496, Wikipedia:Ascending_aorta Relationships: is a type of anatomical structure morphogenesis [GO:0009653]; is part of ascending aorta development [GO:0035905]; is part of aorta morphogenesis [GO:0035909] Definition: The process in which the anatomical structures of the ascending aorta are generated and organized. The ascending aorta is the portion of the aorta in a two-pass circulatory system that lies between the heart and the arch of aorta. In a two-pass circulatory system blood passes twice through the heart to supply the body once.